{
  "gene_symbol": "DXO",
  "gene": "UniProtKB:O77932",
  "term_label": "mRNA 5'-diphosphatase activity",
  "term_id": "GO:0034353",
  "gene_name": "Decapping and exoribonuclease protein"
}